thiamine-containing compound metabolic process [GO:0042723] (biological process) Subtypes: GO:0006772, thiamine diphosphate metabolic process [GO:0042357], thiamine-containing compound biosynthetic process [GO:0042724], thiamine-containing compound catabolic process [GO:0042725] Also known as: thiamin and derivative metabolic process, thiamin and derivative metabolism, thiamin-containing compound metabolic process, thiamine and derivative metabolic process, thiamine and derivative metabolism, thiamine-containing compound metabolism, vitamin B1 and derivative metabolic process, vitamin B1 and derivative metabolism Definition: The chemical reactions and pathways involving thiamine (vitamin B1), and compounds derived from it. Sources: GOC:jl Relationships: is a type of sulfur compound metabolic process [GO:0006790]; is a type of pyrimidine-containing compound metabolic process [GO:0072527]